{
  "gene_name": "Secretory carrier-associated membrane protein 1",
  "term_id": "GO:0032588",
  "gene": "UniProtKB:O15126",
  "gene_symbol": "SCAMP1",
  "term_label": "trans-Golgi network membrane"
}